{
  "gene": "UniProtKB:Q9UGQ2",
  "gene_name": "Calcium channel flower homolog",
  "gene_symbol": "CACFD1",
  "term_label": "vesicle-mediated transport",
  "term_id": "GO:0016192"
}